{
  "gene_name": "BPI fold-containing family B member 3",
  "term_id": "UNKNOWN:0002",
  "gene": "UniProtKB:P59826",
  "gene_symbol": "BPIFB3",
  "term_label": "Unknown biological process"
}